negative regulation of asperthecin biosynthetic process [GO:1900380] (biological process) Sources: GOC:TermGenie, GOC:di Definition: Any process that stops, prevents or reduces the frequency, rate or extent of asperthecin biosynthetic process. Also known as: down regulation of asperthecin biosynthesis, down regulation of asperthecin biosynthetic process, down regulation of asperthecin formation, down regulation of asperthecin synthesis, down-regulation of asperthecin biosynthesis, down-regulation of asperthecin biosynthetic process, down-regulation of asperthecin formation, down-regulation of asperthecin synthesis, downregulation of asperthecin biosynthesis, downregulation of asperthecin biosynthetic process, downregulation of asperthecin formation, downregulation of asperthecin synthesis, inhibition of asperthecin biosynthesis, inhibition of asperthecin formation, inhibition of asperthecin synthesis, negative regulation of asperthecin biosynthesis, negative regulation of asperthecin formation, negative regulation of asperthecin synthesis, inhibition of asperthecin biosynthetic process Relationships: is a type of negative regulation of small molecule metabolic process [GO:0062014]; is a type of negative regulation of secondary metabolite biosynthetic process [GO:1900377]; is a type of regulation of asperthecin biosynthetic process [GO:1900379]; negatively regulates GO:0036184